{
  "term_label": "Unknown molecular function",
  "gene": "UniProtKB:Q9H9A6",
  "gene_symbol": "LRRC40",
  "gene_name": "Leucine-rich repeat-containing protein 40",
  "term_id": "UNKNOWN:0001"
}